desmosome maintenance [GO:0002160] (biological process) Relationships: is a type of desmosome organization [GO:0002934]; is a type of GO:0045217 Definition: The maintenance of a desmosome. A desmosome is a patch-like intercellular junctions found in vertebrate tissues, consisting of parallel zones of two cell membranes, separated by an interspace of 25-35 nm, and having dense fibrillar plaques in the subjacent cytoplasm. Note: Desmosomes link two cells together; hemidesmosomes attach one cell to the extracellular matrix. Sources: GOC:hjd, ISBN:0198506732